{
  "gene": "UniProtKB:P41970",
  "gene_name": "ETS domain-containing protein Elk-3",
  "gene_symbol": "ELK3",
  "term_label": "DNA-binding transcription factor activity, RNA polymerase II-specific",
  "term_id": "GO:0000981"
}